ciliary shaft [GO:0097544] (cellular component) Note: Note that 'ciliary shaft' is sparingly used in the literature to denote the projecting part of the cilium; many authors would refer to the axoneme instead. However, the definition of GO:0005930 'axoneme' is rather stringent, and the localization of many ciliary proteins would not fit that definition. Also, note that cilia and eukaryotic flagella are deemed to be equivalent. Definition: The mid part of a cilium between the ciliary base and ciliary tip that extends into the extracellular space. References: PMID:19866682 Sources: GOC:cilia, GOC:krc Also known as: cilial shaft, cilium shaft, flagellar shaft, flagellum shaft Relationships: is a type of cellular anatomical structure [GO:0110165]; is part of cilium [GO:0005929]; has part axoneme [GO:0005930]